{
  "gene_symbol": "DEFA3",
  "gene_name": "Neutrophil defensin 3",
  "term_label": "disruption of plasma membrane integrity in another organism",
  "gene": "UniProtKB:P59666",
  "term_id": "GO:0051673"
}